meiotic strand displacement involved in double-strand break repair via SDSA [GO:1902346] (biological process) References: PMID:22723423 Sources: GOC:TermGenie, GOC:al Relationships: is a type of meiotic strand displacement [GO:0000714]; is part of GO:0045003 Also known as: meiotic strand displacement involved in SDSA, meiotic strand displacement involved in double-strand break repair via synthesis-dependent strand annealing, meiotic D-loop dissociation involved in double-strand break repair via synthesis-dependent strand annealing, meiotic D-loop dissociation involved in mitotic gene conversion, meiotic D-loop processing involved in double-strand break repair via synthesis-dependent strand annealing, meiotic D-loop processing involved in mitotic gene conversion, meiotic displacement loop dissociation involved in double-strand break repair via synthesis-dependent strand annealing, meiotic displacement loop dissociation involved in mitotic gene conversion, meiotic displacement loop processing involved in double-strand break repair via synthesis-dependent strand annealing, meiotic displacement loop processing involved in mitotic gene conversion, meiotic strand displacement involved in mitotic gene conversion Definition: Any meiotic strand displacement that is involved in double-strand break repair via synthesis-dependent strand annealing (SDSA).